{
  "term_label": "olfactory receptor activity",
  "gene_name": "Olfactory receptor 5G3",
  "gene_symbol": "OR5G3",
  "gene": "UniProtKB:P0C626",
  "term_id": "GO:0004984"
}